{
  "gene_name": "Autophagy-related protein 2 homolog A",
  "term_label": "phagophore assembly site",
  "term_id": "GO:0000407",
  "gene_symbol": "ATG2A",
  "gene": "UniProtKB:Q2TAZ0"
}